{
  "term_id": "GO:0006886",
  "gene": "UniProtKB:P61923",
  "gene_name": "Coatomer subunit zeta-1",
  "gene_symbol": "COPZ1",
  "term_label": "intracellular protein transport"
}